{
  "term_id": "UNKNOWN:0003",
  "gene": "UniProtKB:Q86VX2",
  "term_label": "Unknown cellular component",
  "gene_name": "COMM domain-containing protein 7",
  "gene_symbol": "COMMD7"
}